histone H4K20me2 reader activity [GO:0140005] (molecular function) Also known as: H4K20me2 modified histone binding Relationships: is a type of histone H4 reader activity [GO:0140008] References: PMID:22150589 Note: Note that the residue position corresponds to the canonical human H4 histone (UniProtKB:P02309); this residue is conserved across all eukaryotes. Note that the initiation methionine is cleaved, so the first residue is S1. Definition: A histone reader that recognizes a histone H4 dimethylated at lysine 20.